{
  "term_label": "Unknown molecular function",
  "gene": "UniProtKB:C9JQI7",
  "gene_name": "Transmembrane protein 232",
  "term_id": "UNKNOWN:0001",
  "gene_symbol": "TMEM232"
}